{
  "gene_symbol": "ARHGAP11B",
  "term_id": "UNKNOWN:0003",
  "gene_name": "Inactive Rho GTPase-activating protein 11B",
  "term_label": "Unknown cellular component",
  "gene": "UniProtKB:Q3KRB8"
}